negative regulation of long-chain fatty acid import into cell [GO:0140213] (biological process) References: PMID:28178239 Definition: Any process that stops, prevents or reduces the frequency, rate or extent of long-chain fatty acid import into a cell. Subtypes: negative regulation of long-chain fatty acid import across plasma membrane [GO:0010748] Relationships: is a type of regulation of long-chain fatty acid import into cell [GO:0140212]; is a type of GO:2000192; negatively regulates long-chain fatty acid import into cell [GO:0044539]